{
  "term_label": "Unknown biological process",
  "gene_name": "PX domain-containing protein 1",
  "gene": "UniProtKB:Q5TGL8",
  "gene_symbol": "PXDC1",
  "term_id": "UNKNOWN:0002"
}